{
  "gene": "UniProtKB:O75711",
  "gene_symbol": "SCRG1",
  "term_label": "neuron projection terminus",
  "term_id": "GO:0044306",
  "gene_name": "Scrapie-responsive protein 1"
}